single thymine insertion binding [GO:0032143] (MF) Sources: GOC:mah, GOC:vk Definition: Binding to a double-stranded DNA region containing a single thymine insertion or a deletion that results in an unpaired thymine. Relationships: is a type of GO:0032138